D-xylulose 5-phosphate biosynthetic process [GO:1901159] (biological process) Definition: The chemical reactions and pathways resulting in the formation of D-xylulose 5-phosphate. Also known as: xylulose 5-phosphate anabolism, xylulose 5-phosphate biosynthesis, xylulose 5-phosphate formation, xylulose 5-phosphate synthesis Sources: GOC:TermGenie, GOC:bf Relationships: is a type of D-xylulose 5-phosphate metabolic process [GO:0051167]; is a type of organophosphate biosynthetic process [GO:0090407]; is_a carbohydrate derivative biosynthetic process [GO:1901137]